{
  "term_label": "calcium ion binding",
  "gene_symbol": "DSG2",
  "term_id": "GO:0005509",
  "gene_name": "Desmoglein-2",
  "gene": "UniProtKB:Q14126"
}